{
  "term_label": "chromatin",
  "gene_name": "Lysine-specific demethylase 5D",
  "gene_symbol": "KDM5D",
  "term_id": "GO:0000785",
  "gene": "UniProtKB:Q9BY66"
}